acridine:proton antiporter activity [GO:0042962] (molecular function) Relationships: is a type of proton transmembrane transporter activity [GO:0015078]; is a type of GO:0015297 References: PMID:10735876 Also known as: acridine:hydrogen antiporter activity, acridine efflux pump activity Definition: Enables the transfer of a solute or solutes from one side of a membrane to the other according to the reaction: H+(out) + acridine(in) = H+(in) + acridine(out).